{
  "gene_name": "Reticulophagy regulator 2",
  "term_id": "UNKNOWN:0002",
  "gene": "UniProtKB:Q8NC44",
  "term_label": "Unknown biological process",
  "gene_symbol": "RETREG2"
}